{
  "term_id": "GO:0005886",
  "gene": "UniProtKB:Q04609",
  "gene_name": "Glutamate carboxypeptidase 2",
  "gene_symbol": "FOLH1",
  "term_label": "plasma membrane"
}